positive regulation of cAMP/PKA signal transduction [GO:0141163] (biological process) Relationships: is a type of regulation of cAMP/PKA signal transduction [GO:0141161]; is a type of positive regulation of intracellular signal transduction [GO:1902533]; positively regulates cAMP/PKA signal transduction [GO:0141156] Also known as: positive regulation of cAMP/PKA signaling References: PMID:21585352 Definition: Any process that activates or increases the frequency, rate or extent of cAMP/PKA signal transduction.